{
  "term_id": "GO:0008467",
  "term_label": "[heparan sulfate]-glucosamine 3-sulfotransferase activity",
  "gene_name": "Heparan sulfate glucosamine 3-O-sulfotransferase 3A1",
  "gene": "UniProtKB:Q9Y663",
  "gene_symbol": "HS3ST3A1"
}